active borate transmembrane transporter activity [GO:0046715] (molecular function) References: PMID:12447444 Relationships: is a type of active transmembrane transporter activity [GO:0022804]; is part of borate transmembrane transport [GO:0035445] Also known as: borate transmembrane transporter activity, efflux-type borate transporter, borate uptake transmembrane transporter activity, boron transmembrane transporter activity, boron uptake transmembrane transporter activity, efflux-type boron transporter Definition: Enables the transport of borate across a membrane against the concentration gradient.